{
  "gene": "UniProtKB:Q149N8",
  "gene_symbol": "SHPRH",
  "gene_name": "E3 ubiquitin-protein ligase SHPRH",
  "term_id": "GO:0000209",
  "term_label": "protein polyubiquitination"
}